{
  "term_id": "GO:0045211",
  "term_label": "postsynaptic membrane",
  "gene_name": "Potassium voltage-gated channel subfamily C member 1",
  "gene_symbol": "KCNC1",
  "gene": "UniProtKB:P48547"
}